{
  "gene_symbol": "MYOF",
  "term_id": "GO:0046928",
  "gene": "UniProtKB:Q9NZM1",
  "term_label": "regulation of neurotransmitter secretion",
  "gene_name": "Myoferlin"
}